{
  "gene": "UniProtKB:Q6ZNE9",
  "gene_symbol": "RUFY4",
  "gene_name": "RUN and FYVE domain-containing protein 4",
  "term_label": "phosphatidylinositol-3-phosphate binding",
  "term_id": "GO:0032266"
}